rhombomere cell migration [GO:0022035] (biological process) Relationships: is_a GO:0021535; is part of rhombomere development [GO:0021546] Definition: The movement of a cell within a rhombomere. This process is known to occur as an early step in the generation of anatomical structure from a rhombomere. References: PMID:15629700 Sources: GOC:cls, GOC:dgh, GOC:dph, GOC:jid, GO_REF:0000021